{
  "gene": "UniProtKB:P35372",
  "term_label": "beta-endorphin receptor activity",
  "term_id": "GO:0004979",
  "gene_name": "Mu-type opioid receptor",
  "gene_symbol": "OPRM1"
}